{
  "gene_symbol": "GABARAPL3",
  "gene": "UniProtKB:Q9BY60",
  "gene_name": "Gamma-aminobutyric acid receptor-associated protein-like 3",
  "term_id": "GO:0050811",
  "term_label": "GABA receptor binding"
}